negative regulation of pseudohyphal septin ring assembly [GO:0062166] (BP) References: PMID:29567712 Definition: Any process that decreases the rate, frequency or extent of pseudohyphal septin ring assembly. Relationships: is a type of negative regulation of protein-containing complex assembly [GO:0031333]; is a type of GO:0051494; is a type of GO:0062164; is a type of GO:1902116; negatively regulates pseudohyphal septin ring assembly [GO:0062163]